{
  "term_id": "GO:0005615",
  "gene_symbol": "GREM2",
  "gene_name": "Gremlin-2",
  "term_label": "extracellular space",
  "gene": "UniProtKB:Q9H772"
}